mitochondrial ATP-gated potassium channel activity [GO:0062156] (molecular function) Also known as: mitoK-ATP activity, mitochondrial potassium channel activity Definition: Enables the ATP-dependent diffusion of a potassium ion across the mitochondrial inner membrane. Relationships: is a type of potassium channel activity [GO:0005267]; is a type of ATP-gated ion channel activity [GO:0035381]; is a type of GO:0099094 References: PMID:31435016